dichotomous subdivision of terminal units involved in ureteric bud branching [GO:0060678] (biological process) Also known as: bifid subdivision of terminal units involved in ureteric bud branching References: PMID:16916378 Sources: GOC:dph Definition: The process in which a ureteric bud bifurcates at its end. Relationships: is_a dichotomous subdivision of an epithelial terminal unit [GO:0060600]; is part of branching involved in ureteric bud morphogenesis [GO:0001658]